myosin I head/neck binding [GO:0032031] (molecular function) Definition: Binding to the head/neck region of a myosin I heavy chain. Sources: GOC:mah Relationships: is a type of myosin head/neck binding [GO:0032028]; is a type of myosin I heavy chain binding [GO:0032037]